synaptic vesicle lumen acidification [GO:0097401] (biological process) Regulation: regulated by regulation of synaptic vesicle lumen acidification [GO:1901546]; negatively regulated by negative regulation of synaptic vesicle lumen acidification [GO:1901547]; positively regulated by GO:1901548 References: PMID:21172605, PMID:22875945 Sources: GOC:dsf Relationships: is a type of establishment of localization in cell [GO:0051649]; is a type of neuron cellular homeostasis [GO:0070050]; is a type of proton transmembrane transport [GO:1902600]; is part of GO:0016188; is part of GO:0099504 Also known as: synaptic vesicle lumen pH reduction, synaptic vesicle proton loading Definition: The acidification of the synaptic vesicle lumen via transport of protons into the vesicle. The resulting electrochemical gradient powers neurotransmitter loading.